{
  "term_id": "GO:1990809",
  "gene_symbol": "RTN4",
  "gene_name": "Reticulon-4",
  "term_label": "endoplasmic reticulum tubular network membrane organization",
  "gene": "UniProtKB:Q9NQC3"
}